membrane tag activity [GO:0141048] (molecular function) Relationships: is a type of GO:0141047 Definition: A molecular function exhibited by a protein that is covalently attached (AKA tagged or conjugated) to a lipid, where it acts as a marker for a membrane, recognized by the cellular apparatus to target the tagged protein for some cellular process such as autophagy. References: PMID:17632063 Also known as: covalent modifier, lipid tag Note: Use this term to annotate conjugated tags, not for conjugating enzymes. At the time of writing, all known gene products with this activity are ubiquitin-like, either based on overall sequence similarity or the presence of common motifs and structures.